{
  "gene_name": "Uncharacterized protein C6orf62",
  "gene_symbol": "C6orf62",
  "term_label": "Unknown molecular function",
  "gene": "UniProtKB:Q9GZU0",
  "term_id": "UNKNOWN:0001"
}